{
  "gene_symbol": "SMIM26",
  "gene": "UniProtKB:A0A096LP01",
  "term_label": "mitochondrion",
  "gene_name": "Small integral membrane protein 26",
  "term_id": "GO:0005739"
}